{
  "gene_symbol": "PGGT1B",
  "gene": "UniProtKB:P53609",
  "term_label": "CAAX-protein geranylgeranyltransferase activity",
  "term_id": "GO:0004662",
  "gene_name": "Geranylgeranyl transferase type-1 subunit beta"
}